{
  "gene_symbol": "NDUFA5",
  "term_label": "Unknown molecular function",
  "gene": "UniProtKB:Q16718",
  "term_id": "UNKNOWN:0001",
  "gene_name": "NADH dehydrogenase [ubiquinone] 1 alpha subcomplex subunit 5"
}